rubrospinal tract morphogenesis [GO:0021964] (biological process) Relationships: is a type of central nervous system projection neuron axonogenesis [GO:0021952] Definition: Generation of a long process of a CNS neuron, that carries efferent (outgoing) action potentials from the cell body in the red nucleus of the midbrain towards target cells in the spinal cord. Sources: GOC:cls, GOC:dgh, GOC:dph, GOC:jid, GO_REF:0000021